{
  "gene_name": "Arrestin domain-containing protein 3",
  "gene": "UniProtKB:Q96B67",
  "term_label": "Unknown biological process",
  "gene_symbol": "ARRDC3",
  "term_id": "UNKNOWN:0002"
}